{
  "gene_name": "Glyceraldehyde-3-phosphate dehydrogenase, testis-specific",
  "gene": "UniProtKB:O14556",
  "term_id": "GO:0006096",
  "term_label": "glycolytic process",
  "gene_symbol": "GAPDHS"
}